{
  "gene": "UniProtKB:P04141",
  "term_label": "cytokine activity",
  "term_id": "GO:0005125",
  "gene_symbol": "CSF2",
  "gene_name": "Granulocyte-macrophage colony-stimulating factor"
}